dehydrogluconate dehydrogenase activity [GO:0047843] (molecular function) Sources: RHEA:12368 Also known as: 2-dehydro-D-gluconate:acceptor 2-oxidoreductase activity, 2-keto-D-gluconate dehydrogenase activity, 2-oxogluconate dehydrogenase activity, alpha-ketogluconate dehydrogenase activity, ketogluconate dehydrogenase activity Relationships: is a type of oxidoreductase activity, acting on CH-OH group of donors [GO:0016614] Definition: Catalysis of the reaction: 2-dehydro-D-gluconate + A = 2,5-didehydro-D-gluconate + AH(2).